{
  "term_label": "olfactory receptor activity",
  "term_id": "GO:0004984",
  "gene": "UniProtKB:A3KFT3",
  "gene_symbol": "OR2M5",
  "gene_name": "Olfactory receptor 2M5"
}